propylene catabolic process [GO:0042208] (biological process) Sources: GOC:jl Relationships: is_a propylene metabolic process [GO:0018964]; is a type of xenobiotic catabolic process [GO:0042178]; is a type of alkene catabolic process [GO:0043451] Definition: The chemical reactions and pathways resulting in the breakdown of propylene, an alkene produced by catalytic or thermal cracking of hydrocarbons or as a by-product of petroleum refining. Also known as: propylene breakdown, propylene catabolism, propylene degradation